specification of plant organ identity [GO:0090701] (biological process) Definition: The regionalization process in which the identity of a plant organ primordium is specified. Identity is considered to be the aggregate of characteristics by which a structure is recognized. Sources: GOC:tb Relationships: is a type of regionalization [GO:0003002]; is part of plant organ formation [GO:1905393] Subtypes: specification of floral organ identity [GO:0010093]